{
  "gene_name": "F-box_WD repeat-containing protein 12",
  "gene": "UniProtKB:Q6X9E4",
  "term_label": "Unknown molecular function",
  "gene_symbol": "FBXW12",
  "term_id": "UNKNOWN:0001"
}